nuclear-transcribed mRNA catabolic process [GO:0000956] (BP) Definition: The chemical reactions and pathways resulting in the breakdown of nuclear-transcribed mRNAs in eukaryotic cells. Relationships: is a type of mRNA catabolic process [GO:0006402] Sources: GOC:krc Also known as: nuclear mRNA breakdown, nuclear mRNA catabolism, nuclear mRNA degradation Subtypes: nuclear-transcribed mRNA catabolic process, nonsense-mediated decay [GO:0000184], nuclear-transcribed mRNA catabolic process, deadenylation-dependent decay [GO:0000288], GO:0000289, GO:0000290, GO:0000294, nuclear-transcribed mRNA catabolic process, deadenylation-independent decay [GO:0031086], nuclear-transcribed mRNA catabolic process, non-stop decay [GO:0070481], nuclear-transcribed mRNA catabolic process, no-go decay [GO:0070966], GO:0071028, histone mRNA catabolic process [GO:0071044]